{
  "gene": "UniProtKB:P02748",
  "gene_name": "Complement component C9",
  "term_label": "complement activation",
  "term_id": "GO:0006956",
  "gene_symbol": "C9"
}